{
  "gene": "UniProtKB:Q9NQT6",
  "gene_symbol": "FSCN3",
  "term_label": "lamellipodium",
  "gene_name": "Fascin-3",
  "term_id": "GO:0030027"
}